female urethra development [GO:0061070] (biological process) Sources: GOC:dph Definition: The progression of the female urethra over time from its initial formation to the mature structure. The female urethra is a renal system organ that carries urine from the bladder to outside the body, exiting above the vaginal opening. Relationships: is a type of urethra development [GO:0061068]